{
  "gene_symbol": "REV1",
  "gene": "UniProtKB:Q9UBZ9",
  "term_id": "GO:0060090",
  "term_label": "molecular adaptor activity",
  "gene_name": "DNA repair protein REV1"
}